{
  "term_label": "Unknown cellular component",
  "gene": "UniProtKB:O75971",
  "gene_name": "snRNA-activating protein complex subunit 5",
  "term_id": "UNKNOWN:0003",
  "gene_symbol": "SNAPC5"
}